metalloaminopeptidase activity [GO:0070006] (molecular function) Relationships: is a type of aminopeptidase activity [GO:0004177]; is a type of metalloexopeptidase activity [GO:0008235] Sources: https://www.ebi.ac.uk/merops/about/glossary.shtml#AMINOPEPTIDASE Definition: Catalysis of the hydrolysis of a single N-terminal amino acid residue from a polypeptide chain by a mechanism in which water acts as a nucleophile, one or two metal ions hold the water molecule in place, and charged amino acid side chains are ligands for the metal ions.